{
  "term_id": "GO:0031267",
  "gene_name": "Dedicator of cytokinesis protein 1",
  "gene_symbol": "DOCK1",
  "term_label": "small GTPase binding",
  "gene": "UniProtKB:Q14185"
}